{
  "term_label": "Unknown molecular function",
  "gene": "UniProtKB:Q04941",
  "term_id": "UNKNOWN:0001",
  "gene_symbol": "PLP2",
  "gene_name": "Proteolipid protein 2"
}